{
  "gene_symbol": "INCA1",
  "term_id": "GO:0008285",
  "gene": "UniProtKB:Q0VD86",
  "gene_name": "Protein INCA1",
  "term_label": "negative regulation of cell population proliferation"
}